{
  "term_label": "nucleus",
  "gene_name": "Cyclin-dependent kinase 4 inhibitor C",
  "gene": "UniProtKB:P42773",
  "term_id": "GO:0005634",
  "gene_symbol": "CDKN2C"
}